{
  "gene_symbol": "CHORDC1",
  "term_label": "Unknown cellular component",
  "gene": "UniProtKB:Q9UHD1",
  "term_id": "UNKNOWN:0003",
  "gene_name": "Cysteine and histidine-rich domain-containing protein 1"
}